{
  "gene_symbol": "SCAMP4",
  "term_label": "exocytosis",
  "gene_name": "Secretory carrier-associated membrane protein 4",
  "term_id": "GO:0006887",
  "gene": "UniProtKB:Q969E2"
}